{
  "gene_name": "Acyl-coenzyme A synthetase ACSM1, mitochondrial",
  "gene": "UniProtKB:Q08AH1",
  "gene_symbol": "ACSM1",
  "term_label": "mitochondrial matrix",
  "term_id": "GO:0005759"
}